{
  "term_id": "GO:0001963",
  "term_label": "synaptic transmission, dopaminergic",
  "gene_name": "Adenosine receptor A2a",
  "gene_symbol": "ADORA2A",
  "gene": "UniProtKB:P29274"
}